{
  "term_label": "actin cytoskeleton organization",
  "gene": "UniProtKB:O00401",
  "gene_symbol": "WASL",
  "gene_name": "Actin nucleation-promoting factor WASL",
  "term_id": "GO:0030036"
}